synaptotagmin-synaptobrevin 2-SNAP-25-syntaxin-1a-syntaxin-1b-Unc13 complex [GO:0070768] (cellular component) Relationships: is a type of SNARE complex [GO:0031201] Definition: A SNARE complex that contains synaptotagmin, synaptobrevin 2 (VAMP2), SNAP-25, syntaxin 1a, syntaxin1b, and Unc13b (or orthologs thereof). References: PMID:8999968 Also known as: SNARE complex (Snap25, Syt1, Unc13b, Vamp2, Stx1b2, Stx1a), Snap25-Syt1-Unc13b-Vamp2-Stx1b2-Stx1a complex